{
  "gene_symbol": "NAA15",
  "gene_name": "N-alpha-acetyltransferase 15, NatA auxiliary subunit",
  "gene": "UniProtKB:Q9BXJ9",
  "term_label": "acetyltransferase activator activity",
  "term_id": "GO:0010698"
}